{
  "term_id": "GO:0038187",
  "gene_symbol": "CLEC17A",
  "term_label": "pattern recognition receptor activity",
  "gene_name": "C-type lectin domain family 17, member A",
  "gene": "UniProtKB:Q6ZS10"
}